regulation of intestinal D-glucose absorption [GO:1903985] (biological process) Definition: Any process that modulates the frequency, rate or extent of intestinal D-glucose absorption. References: PMID:22114352 Sources: GOA:als, GOC:TermGenie, GO_REF:0000058 Relationships: is a type of GO:1904478; regulates intestinal D-glucose absorption [GO:0001951]